regulation of osteoblast differentiation [GO:0045667] (BP) Definition: Any process that modulates the frequency, rate or extent of osteoblast differentiation. Sources: GOC:go_curators Relationships: is_a regulation of cell differentiation [GO:0045595]; regulates osteoblast differentiation [GO:0001649] Subtypes: GO:0045668, positive regulation of osteoblast differentiation [GO:0045669]